gluconate 2-dehydrogenase (acceptor) activity [GO:0033717] (molecular function) Also known as: 2-ketogluconate reductase activity, D-gluconate dehydrogenase activity, D-gluconate dehydrogenase, 2-keto-D-gluconate-yielding activity, D-gluconate:(acceptor) 2-oxidoreductase activity, D-gluconate:acceptor 2-oxidoreductase activity, gluconate oxidase activity, gluconic acid dehydrogenase activity, gluconic dehydrogenase activity Definition: Catalysis of the reaction: D-gluconate + acceptor = 2-dehydro-D-gluconate + reduced acceptor. Sources: RHEA:12769 Relationships: is a type of gluconate dehydrogenase activity [GO:0008875]